{
  "gene": "UniProtKB:Q9BYX4",
  "term_label": "zinc ion binding",
  "term_id": "GO:0008270",
  "gene_name": "Interferon-induced helicase C domain-containing protein 1",
  "gene_symbol": "IFIH1"
}